voltage-gated sodium channel complex [GO:0001518] (cellular component) Definition: A sodium channel in a cell membrane whose opening is governed by the membrane potential. Sources: ISBN:0198506732 Also known as: voltage gated sodium channel complex, voltage-dependent sodium channel complex, voltage-sensitive sodium channel complex Relationships: is_a sodium channel complex [GO:0034706]; is a type of plasma membrane protein complex [GO:0098797]